{
  "gene": "UniProtKB:Q8NCL8",
  "gene_name": "Transmembrane protein 116",
  "gene_symbol": "TMEM116",
  "term_label": "Unknown biological process",
  "term_id": "UNKNOWN:0002"
}